{
  "gene_symbol": "PTEN",
  "gene": "UniProtKB:P60484",
  "gene_name": "Phosphatidylinositol 3,4,5-trisphosphate 3-phosphatase and dual-specificity protein phosphatase PTEN",
  "term_id": "GO:0004725",
  "term_label": "protein tyrosine phosphatase activity"
}